{
  "gene_name": "Sperm-associated antigen 17",
  "term_label": "epithelial cilium movement involved in extracellular fluid movement",
  "term_id": "GO:0003351",
  "gene": "UniProtKB:Q6Q759",
  "gene_symbol": "SPAG17"
}